{
  "term_id": "GO:0004984",
  "gene": "UniProtKB:Q8NH64",
  "gene_name": "Olfactory receptor 51A7",
  "gene_symbol": "OR51A7",
  "term_label": "olfactory receptor activity"
}